extraction of mislocalized protein from ER membrane [GO:0140569] (biological process) References: PMID:32973005 Relationships: is_a GO:0140568 Definition: The removal of a mislocalized protein from the endoplasmic reticulum (ER) membrane.